{
  "gene_name": "Guanine nucleotide-binding protein G(I)_G(S)_G(O) subunit gamma-10",
  "gene": "UniProtKB:P50151",
  "term_id": "GO:0005834",
  "gene_symbol": "GNG10",
  "term_label": "heterotrimeric G-protein complex"
}